{
  "gene_symbol": "DBH",
  "term_label": "dopamine catabolic process",
  "gene": "UniProtKB:P09172",
  "term_id": "GO:0042420",
  "gene_name": "Dopamine beta-hydroxylase"
}